{
  "gene_name": "T cell receptor beta joining 2-7",
  "gene_symbol": "TRBJ2-7",
  "term_id": "UNKNOWN:0002",
  "gene": "UniProtKB:A0A0A0MT78",
  "term_label": "Unknown biological process"
}